{
  "term_id": "GO:0007411",
  "gene_name": "Semaphorin-6A",
  "gene": "UniProtKB:Q9H2E6",
  "term_label": "axon guidance",
  "gene_symbol": "SEMA6A"
}